{
  "term_label": "vesicle-mediated transport",
  "gene_symbol": "ARF5",
  "gene_name": "ADP-ribosylation factor 5",
  "term_id": "GO:0016192",
  "gene": "UniProtKB:P84085"
}